{
  "gene": "UniProtKB:P24390",
  "term_id": "GO:0046923",
  "gene_symbol": "KDELR1",
  "gene_name": "ER lumen protein-retaining receptor 1",
  "term_label": "ER retention sequence binding"
}